{
  "gene_name": "Actin-associated protein FAM107A",
  "gene": "UniProtKB:O95990",
  "gene_symbol": "FAM107A",
  "term_id": "GO:0001725",
  "term_label": "stress fiber"
}